{
  "term_id": "GO:0005096",
  "gene": "UniProtKB:P52757",
  "gene_name": "Beta-chimaerin",
  "gene_symbol": "CHN2",
  "term_label": "GTPase activator activity"
}